{
  "gene": "UniProtKB:P11279",
  "term_label": "Unknown molecular function",
  "gene_symbol": "LAMP1",
  "gene_name": "Lysosome-associated membrane glycoprotein 1",
  "term_id": "UNKNOWN:0001"
}